{
  "term_id": "UNKNOWN:0002",
  "gene_name": "Ankyrin repeat and SOCS box protein 10",
  "gene": "UniProtKB:Q8WXI3",
  "term_label": "Unknown biological process",
  "gene_symbol": "ASB10"
}